pinosome [GO:0044352] (cellular component) Relationships: is a type of GO:0005768 References: PMID:14731589, PMID:14732047 Also known as: pinocytic vesicle Definition: A membrane-bounded, uncoated intracellular vesicle formed by the process of pinocytosis. Subtypes: GO:0044353, GO:0044354